{
  "term_label": "protein tyrosine phosphatase activity",
  "gene": "UniProtKB:P23469",
  "gene_symbol": "PTPRE",
  "gene_name": "Receptor-type tyrosine-protein phosphatase epsilon",
  "term_id": "GO:0004725"
}